{
  "term_id": "UNKNOWN:0001",
  "term_label": "Unknown molecular function",
  "gene": "UniProtKB:Q5T5J6",
  "gene_name": "Transcriptional protein SWT1",
  "gene_symbol": "SWT1"
}